{
  "gene_name": "Putative ribosomal protein eL43-like",
  "term_label": "cytosolic large ribosomal subunit",
  "gene_symbol": "RPL37AP8",
  "term_id": "GO:0022625",
  "gene": "UniProtKB:A6NKH3"
}